regulation of lateral attachment of mitotic spindle microtubules to kinetochore [GO:1905115] (biological process) Relationships: is a type of regulation of attachment of mitotic spindle microtubules to kinetochore [GO:1902423]; regulates lateral attachment of mitotic spindle microtubules to kinetochore [GO:0099607] Definition: Any process that modulates the frequency, rate or extent of lateral attachment of mitotic spindle microtubules to kinetochore. References: PMID:22375062 Sources: GOC:TermGenie, GO_REF:0000058 Subtypes: GO:1905116